{
  "gene": "UniProtKB:A0A1B0GTU1",
  "gene_name": "Zinc finger CCCH domain-containing protein 11B",
  "term_id": "GO:0005634",
  "term_label": "nucleus",
  "gene_symbol": "ZC3H11B"
}